{
  "term_id": "UNKNOWN:0001",
  "gene_symbol": "SDC3",
  "gene_name": "Syndecan-3",
  "term_label": "Unknown molecular function",
  "gene": "UniProtKB:O75056"
}